{
  "gene": "UniProtKB:P16220",
  "term_id": "GO:0035497",
  "gene_symbol": "CREB1",
  "gene_name": "Cyclic AMP-responsive element-binding protein 1",
  "term_label": "cAMP response element binding"
}